negative regulation of low-density lipoprotein particle clearance [GO:0010989] (biological process) Relationships: is a type of negative regulation of lipoprotein particle clearance [GO:0010985]; is a type of regulation of low-density lipoprotein particle clearance [GO:0010988]; negatively regulates GO:0034383 Sources: GOC:BHF, GOC:dph, GOC:tb Definition: Any process that decreases the rate, frequency or extent of low-density lipoprotein particle clearance. Low-density lipoprotein particle clearance is the process in which a low-density lipoprotein particle is removed from the blood via receptor-mediated endocytosis and its constituent parts degraded.